{
  "gene_name": "Testis-expressed protein 54",
  "term_id": "UNKNOWN:0001",
  "gene_symbol": "TEX54",
  "term_label": "Unknown molecular function",
  "gene": "UniProtKB:A0A1B0GVG6"
}